negative regulation of bone development [GO:1903011] (biological process) References: PMID:22510437 Sources: GOC:TermGenie, GOC:mr, GO_REF:0000058 Also known as: down regulation of bone development, down-regulation of bone development, downregulation of bone development, inhibition of bone development Definition: Any process that stops, prevents or reduces the frequency, rate or extent of bone development. Relationships: is a type of GO:0051093; is a type of negative regulation of multicellular organismal process [GO:0051241]; is a type of GO:1903010; negatively regulates bone development [GO:0060348]